4-amino-5-hydroxymethyl-2-methylpyrimidine phosphate synthase activity from histidine and PLP [GO:0106344] (molecular function) Definition: Catalysis of the reaction: 2 Fe(3+) + 4 H2O + L-histidyl-[4-amino-5-hydroxymethyl-2-methylpyrimidine phosphate synthase] + N(6)-(pyridoxal phosphate)-L-lysyl-[4-amino-5-hydroxymethyl-2-methylpyrimidine phosphate synthase] = (2S)-2-amino-5-hydroxy-4-oxopentanoyl-[4-amino-5-hydroxymethyl-2-methylpyrimidine phosphate synthase] + 3-oxopropanoate + 4-amino-2-methyl-5-(phosphooxymethyl)pyrimidine + 2 Fe(2+) + 2 H+ + L-lysyl-[4-amino-5-hydroxymethyl-2-methylpyrimidine phosphate synthase]. References: PMID:22568620 Sources: RHEA:65756 Relationships: is_a transferase activity [GO:0016740]